{
  "term_label": "toll-like receptor signaling pathway",
  "term_id": "GO:0002224",
  "gene_symbol": "TIFAB",
  "gene": "UniProtKB:Q6ZNK6",
  "gene_name": "TRAF-interacting protein with FHA domain-containing protein B"
}